ribonucleoside monophosphate catabolic process [GO:0009158] (biological process) Also known as: ribonucleoside monophosphate breakdown, ribonucleoside monophosphate catabolism, ribonucleoside monophosphate degradation Subtypes: purine ribonucleoside monophosphate catabolic process [GO:0009169], pyrimidine ribonucleoside monophosphate catabolic process [GO:0009175], FMN catabolic process [GO:0032363] Sources: GOC:go_curators, ISBN:0198506732 Definition: The chemical reactions and pathways resulting in the breakdown of a ribonucleoside monophosphate, a compound consisting of a nucleobase linked to a ribose sugar esterified with phosphate on the sugar. Relationships: is_a nucleoside monophosphate catabolic process [GO:0009125]